{
  "gene_name": "Protein mono-ADP-ribosyltransferase PARP4",
  "gene": "UniProtKB:Q9UKK3",
  "term_id": "GO:0003950",
  "term_label": "NAD+ poly-ADP-ribosyltransferase activity",
  "gene_symbol": "PARP4"
}